{
  "gene_symbol": "KRTAP6-1",
  "gene": "UniProtKB:Q3LI64",
  "gene_name": "Keratin-associated protein 6-1",
  "term_id": "UNKNOWN:0002",
  "term_label": "Unknown biological process"
}